{
  "term_label": "transcription corepressor activity",
  "gene_symbol": "CIR1",
  "gene": "UniProtKB:Q86X95",
  "gene_name": "Corepressor interacting with RBPJ 1",
  "term_id": "GO:0003714"
}